cytochrome metabolic process [GO:1903604] (biological process) References: PMID:19721088 Sources: GOC:TermGenie, GOC:dph, GO_REF:0000068 Relationships: is a type of protein metabolic process [GO:0019538] Also known as: cytochrome metabolism Definition: The chemical reactions and pathways involving a cytochrome. Subtypes: GO:1903605, cytochrome c metabolic process [GO:1903606]